{
  "gene_name": "Noggin",
  "gene": "UniProtKB:Q13253",
  "term_id": "GO:0005615",
  "term_label": "extracellular space",
  "gene_symbol": "NOG"
}